{
  "term_id": "GO:0003697",
  "gene": "UniProtKB:Q6NSI4",
  "gene_name": "RPA-related protein RADX",
  "term_label": "single-stranded DNA binding",
  "gene_symbol": "RADX"
}